{
  "gene_symbol": "NEK10",
  "gene_name": "Serine_threonine-protein kinase Nek10",
  "term_label": "protein serine/threonine kinase activity",
  "term_id": "GO:0004674",
  "gene": "UniProtKB:Q6ZWH5"
}